renal system segmentation [GO:0061150] (BP) Definition: The regionalization process that divides an the renal system into a series of segments along its proximal/distal axis. Sources: GOC:dph, GOC:yaf Also known as: urinary tract segmentation Relationships: is a type of segmentation [GO:0035282]; is a type of renal system pattern specification [GO:0072048]